{
  "gene": "UniProtKB:O43422",
  "gene_name": "52 kDa repressor of the inhibitor of the protein kinase",
  "gene_symbol": "THAP12",
  "term_label": "Unknown molecular function",
  "term_id": "UNKNOWN:0001"
}